{
  "gene_symbol": "EEF1A1P5",
  "gene": "UniProtKB:Q5VTE0",
  "gene_name": "Putative elongation factor 1-alpha-like 3",
  "term_id": "GO:0006412",
  "term_label": "translation"
}